central complex development [GO:0048036] (biological process) Also known as: central body development Definition: The process whose specific outcome is the progression of the central complex over time, from its formation to the mature structure. The central complex region of the insect brain is thought to be crucial for control of locomotive behavior. Located in the middle of the two protocerebral hemispheres, it comprises four neuropilar regions, the fan-shaped body, the ellipsoid body, the protocerebral bridge and the paired noduli. References: PMID:12490252 Relationships: is a type of anatomical structure development [GO:0048856]; is part of brain development [GO:0007420]